{
  "gene_symbol": "COPG1",
  "term_label": "endoplasmic reticulum to Golgi vesicle-mediated transport",
  "gene": "UniProtKB:Q9Y678",
  "term_id": "GO:0006888",
  "gene_name": "Coatomer subunit gamma-1"
}